{
  "term_id": "GO:0070098",
  "gene_symbol": "XCL1",
  "gene_name": "Lymphotactin",
  "gene": "UniProtKB:P47992",
  "term_label": "chemokine-mediated signaling pathway"
}